protein localization to organelle [GO:0033365] (biological process) Also known as: protein localisation to organelle, protein localization in organelle Relationships: is a type of intracellular protein localization [GO:0008104] Definition: A process in which a protein is transported to, or maintained in, a location within an organelle. Subtypes: GO:0020028, GO:0033366, GO:0034067, protein localization to chromosome [GO:0034502], protein localization to nucleus [GO:0034504], protein localization to endosome [GO:0036010], protein localization to M-band [GO:0036309], protein localization to cytoskeleton [GO:0044380], protein transmembrane import into intracellular organelle [GO:0044743], GO:0061512, ubiquitin-dependent endocytosis [GO:0070086], protein localization to mitochondrion [GO:0070585], protein localization to endoplasmic reticulum [GO:0070972], protein localization to chloroplast [GO:0072598], protein localization to peroxisome [GO:0072662], GO:0072665, protein localization to postsynaptic specialization membrane [GO:0099633], GO:0110012, protein localization to cytoplasmic stress granule [GO:1903608], protein localization to phagocytic vesicle [GO:1905161], protein localization to lipid droplet [GO:1990044] Sources: GOC:mah